{
  "gene": "UniProtKB:B7ZLF3",
  "term_label": "RNA polymerase II cis-regulatory region sequence-specific DNA binding",
  "gene_name": "C2H2-type domain-containing protein",
  "term_id": "GO:0000978",
  "gene_symbol": "LOC728743"
}